mesonephric glomerular epithelium development [GO:0061232] (biological process) Sources: GOC:mtg_kidney_jan10 Relationships: is a type of mesonephric nephron epithelium development [GO:0061241]; is_a glomerular epithelium development [GO:0072010]; is part of GO:0061224 Definition: The process whose specific outcome is the progression of the mesonephric glomerular epithelium over time, from its formation to the mature structure. The mesonephric glomerular epithelium is an epithelial tissue that covers the outer surfaces of the glomerulus in the mesonephros. The mesonephric glomerular epithelium consists of both parietal and visceral epithelium. Mesonephric glomerular parietal epithelial cells are specialized epithelial cells that form tight junctions as a barrier to protein transport. A mesonephric glomerular visceral epithelial cell is a specialized epithelial cell that contains 'feet' that interdigitate with the 'feet' of other glomerular epithelial cells in the mesonephros.